{
  "term_id": "UNKNOWN:0003",
  "gene_name": "Protein IGHD2OR15-2A (Fragment)",
  "gene": "UniProtKB:A0A075B7B9",
  "gene_symbol": "IGHD2OR15-2B",
  "term_label": "Unknown cellular component"
}